NuRD complex [GO:0016581] (cellular component) References: PMID:10589671, PMID:11743021, PMID:17289569 Relationships: is a type of histone deacetylase complex [GO:0000118]; is a type of GO:0005667; is a type of CHD-type complex [GO:0090545] Subtypes: SHREC complex [GO:0070824] Also known as: NRD complex, nucleosome remodeling and histone deacetylation complex, Mi-2 complex Definition: An approximately 2 MDa multi-subunit complex that exhibits ATP-dependent chromatin remodeling activity in addition to histone deacetylase (HDAC) activity, and has been shown to establish transcriptional repression of a number of target genes in vertebrates, invertebrates and fungi. Amongst its subunits, the NuRD complex contains histone deacetylases, histone binding proteins and Mi-2-like proteins.